regulation of dendritic spine development [GO:0060998] (biological process) Definition: Any process that modulates the rate, frequency, or extent of dendritic spine development, the process whose specific outcome is the progression of the dendritic spine over time, from its formation to the mature structure. Sources: GOC:dph Relationships: is_a regulation of developmental process [GO:0050793]; regulates dendritic spine development [GO:0060996] Subtypes: positive regulation of dendritic spine development [GO:0060999], negative regulation of dendritic spine development [GO:0061000]